interleukin-27 receptor activity [GO:0045509] (MF) Definition: Combining with interleukin-27 and transmitting the signal from one side of the membrane to the other to initiate a change in cell activity. Relationships: is a type of GO:0030368; is part of interleukin-27-mediated signaling pathway [GO:0070106]; has part interleukin-27 binding [GO:0045513] Also known as: IL-27 receptor activity, IL-27R Sources: GOC:jl, GOC:signaling